{
  "term_id": "GO:0009653",
  "gene_name": "Forkhead box protein D4-like 1",
  "term_label": "anatomical structure morphogenesis",
  "gene": "UniProtKB:Q9NU39",
  "gene_symbol": "FOXD4L1"
}